{
  "gene_symbol": "TENT2",
  "term_id": "GO:1990817",
  "gene_name": "Poly(A) RNA polymerase GLD2",
  "gene": "UniProtKB:Q6PIY7",
  "term_label": "poly(A) RNA polymerase activity"
}